negative regulation of ribosomal protein gene transcription from RNA polymerase II promoter in response to stress [GO:0010690] (biological process) Definition: Any process that decreases the frequency, rate or extent of the synthesis of RNA from ribosomal protein genes by RNA polymerase II, originating at an RNA polymerase II promoter, as a result of a disturbance in organismal or cellular homeostasis. Sources: GOC:dph, GOC:tb, GOC:txnOH Relationships: is a type of negative regulation of ribosomal protein gene transcription by RNA polymerase II [GO:0010688]; is a type of cellular response to stress [GO:0033554]